exon-exon junction complex [GO:0035145] (cellular component) Subtypes: exon-exon junction subcomplex mago-y14 [GO:1990501] Also known as: EJC, exon junction complex References: PMID:11532962, PMID:11743026 Definition: A multi-subunit complex deposited by the spliceosome upstream of messenger RNA exon-exon junctions. The exon-exon junction complex provides a binding platform for factors involved in mRNA export and nonsense-mediated mRNA decay. Relationships: is_a nuclear protein-containing complex [GO:0140513]